{
  "gene_symbol": "PRXL2A",
  "term_label": "antioxidant activity",
  "term_id": "GO:0016209",
  "gene_name": "Peroxiredoxin-like 2A",
  "gene": "UniProtKB:Q9BRX8"
}